{
  "gene_name": "Coiled-coil domain-containing protein 105",
  "term_id": "UNKNOWN:0001",
  "gene_symbol": "CCDC105",
  "gene": "UniProtKB:Q8IYK2",
  "term_label": "Unknown molecular function"
}